{
  "gene_symbol": "ENO3",
  "gene": "UniProtKB:P13929",
  "gene_name": "Beta-enolase",
  "term_id": "GO:0006096",
  "term_label": "glycolytic process"
}